biotin transmembrane transporter activity [GO:0015225] (molecular function) Also known as: biotin transporter activity, vitamin B7 transporter activity, vitamin H transporter activity Definition: Enables the transfer of biotin from one side of a membrane to the other. Biotin is cis-tetrahydro-2-oxothieno(3,4-d)imidazoline-4-valeric acid; the (+) enantiomer is very widely distributed in cells and serves as a carrier in a number of enzymatic beta-carboxylation reactions. Relationships: is a type of monocarboxylic acid transmembrane transporter activity [GO:0008028]; is a type of amide transmembrane transporter activity [GO:0042887]; is a type of vitamin transmembrane transporter activity [GO:0090482]; is a type of sulfur compound transmembrane transporter activity [GO:1901682]; is part of biotin transport [GO:0015878] Sources: GOC:ai